{
  "term_label": "embryonic pattern specification",
  "gene_name": "Homeobox protein CDX-4",
  "term_id": "GO:0009880",
  "gene_symbol": "CDX4",
  "gene": "UniProtKB:O14627"
}